{
  "gene_symbol": "SIN3A",
  "term_id": "GO:0000122",
  "term_label": "negative regulation of transcription by RNA polymerase II",
  "gene_name": "Paired amphipathic helix protein Sin3a",
  "gene": "UniProtKB:Q96ST3"
}